{
  "gene": "UniProtKB:Q63HN1",
  "term_id": "UNKNOWN:0003",
  "gene_name": "Putative protein SPATA31F2P",
  "gene_symbol": "SPATA31F2P",
  "term_label": "Unknown cellular component"
}